Purkinje myocyte development [GO:0003165] (biological process) Relationships: is a type of GO:0003229; is part of GO:0003164 Also known as: cardiac Purkinje fiber development Sources: GOC:mtg_cardiac_conduct_nov11, GOC:mtg_heart Definition: The process whose specific outcome is the progression of a Purkinje myocyte over time, from its formation to the mature structure. The Purkinje myocyte (also known as cardiac Purkinje fiber) is part of the cardiac conduction system that receives signals from the bundle of His and innervates the ventricular cardiac muscle.